{
  "gene_symbol": "GABRR2",
  "gene": "UniProtKB:P28476",
  "term_label": "chloride channel activity",
  "gene_name": "Gamma-aminobutyric acid receptor subunit rho-2",
  "term_id": "GO:0005254"
}